{
  "gene_symbol": "JRKL",
  "gene": "UniProtKB:Q9Y4A0",
  "gene_name": "Jerky protein homolog-like",
  "term_label": "Unknown biological process",
  "term_id": "UNKNOWN:0002"
}